{
  "term_id": "GO:0009966",
  "term_label": "regulation of signal transduction",
  "gene": "UniProtKB:Q9NZI2",
  "gene_symbol": "KCNIP1",
  "gene_name": "Kv channel-interacting protein 1"
}